ATPase-coupled monoatomic cation transmembrane transporter activity [GO:0019829] (molecular function) Sources: GOC:ai Subtypes: GO:0005388, P-type cadmium transporter activity [GO:0008551], P-type proton-exporting transporter activity [GO:0008553], P-type sodium transporter activity [GO:0008554], GO:0008556, GO:0015408, ABC-type manganese transporter activity [GO:0015410], ABC-type nickel transporter activity [GO:0015413], ABC-type cadmium transporter activity [GO:0015434], GO:0015444, GO:0015445, GO:0015633, P-type zinc transporter activity [GO:0016463], GO:0032778, P-type divalent copper transporter activity [GO:0043682], proton-transporting ATPase activity, rotational mechanism [GO:0046961], sodium-transporting ATPase activity, rotational mechanism [GO:0046962], P-type monovalent copper transporter activity [GO:0140581], GO:0140613, ABC-type sodium transporter activity [GO:0140679] Also known as: ATPase-coupled cation transmembrane transporter activity, ATP-dependent cation transmembrane transporter activity, cation-transporting ATPase activity, cation ABC transporter, plasma membrane cation-transporting ATPase Definition: Enables the transfer of a solute or solutes from one side of a membrane to the other according to the reaction: ATP + H2O + cation(out) = ADP + phosphate + cation(in). Relationships: is a type of monoatomic cation transmembrane transporter activity [GO:0008324]; is a type of active monoatomic ion transmembrane transporter activity [GO:0022853]; is a type of ATPase-coupled transmembrane transporter activity [GO:0042626]